imidazoleglycerol-phosphate synthase complex [GO:0009382] (cellular component) Relationships: is_a transferase complex [GO:1990234]; is part of GO:0005737 Note: See also the molecular function term 'imidazoleglycerol-phosphate synthase activity ; GO:0000107'. Definition: Complex that possesses imidazoleglycerol-phosphate synthase activity. Also known as: imidazoleglycerol phosphate synthase complex Sources: GOC:mah